{
  "term_id": "GO:0005544",
  "gene_name": "Annexin A11",
  "gene": "UniProtKB:P50995",
  "gene_symbol": "ANXA11",
  "term_label": "calcium-dependent phospholipid binding"
}